{
  "gene_symbol": "DTNBP1",
  "gene_name": "Dysbindin",
  "term_id": "GO:0060155",
  "term_label": "platelet dense granule organization",
  "gene": "UniProtKB:Q96EV8"
}